{
  "gene_name": "Solute carrier family 35 member F1",
  "gene_symbol": "SLC35F1",
  "term_label": "Unknown cellular component",
  "term_id": "UNKNOWN:0003",
  "gene": "UniProtKB:Q5T1Q4"
}